{
  "gene": "UniProtKB:Q06547",
  "gene_name": "GA-binding protein subunit beta-1",
  "term_label": "nucleus",
  "term_id": "GO:0005634",
  "gene_symbol": "GABPB1"
}